{
  "gene_name": "Protein mono-ADP-ribosyltransferase PARP14",
  "term_label": "nucleus",
  "gene_symbol": "PARP14",
  "gene": "UniProtKB:Q460N5",
  "term_id": "GO:0005634"
}